structural constituent of postsynaptic specialization [GO:0098879] (molecular function) Definition: The action of a molecule that contributes to the structural integrity of a postsynaptic specialization. Relationships: is a type of GO:0099186; is part of maintenance of postsynaptic specialization structure [GO:0098880]; occurs in GO:0099572 Subtypes: GO:0098919 Sources: GOC:dos